{
  "term_label": "extracellular space",
  "gene_symbol": "GDF6",
  "gene": "UniProtKB:Q6KF10",
  "term_id": "GO:0005615",
  "gene_name": "Growth_differentiation factor 6"
}